{
  "gene": "UniProtKB:Q8IVU3",
  "term_id": "GO:0005737",
  "term_label": "cytoplasm",
  "gene_symbol": "HERC6",
  "gene_name": "Probable E3 ubiquitin-protein ligase HERC6"
}